{
  "term_label": "nucleus",
  "gene_symbol": "FABP9",
  "gene": "UniProtKB:Q0Z7S8",
  "term_id": "GO:0005634",
  "gene_name": "Fatty acid-binding protein 9"
}